{
  "term_id": "GO:0003836",
  "gene_symbol": "ST3GAL1",
  "gene": "UniProtKB:Q11201",
  "term_label": "beta-galactoside (CMP) alpha-2,3-sialyltransferase activity",
  "gene_name": "CMP-N-acetylneuraminate-beta-galactosamide-alpha-2,3-sialyltransferase 1"
}